{
  "term_label": "Unknown molecular function",
  "gene_symbol": "GINS4",
  "gene": "UniProtKB:Q9BRT9",
  "gene_name": "DNA replication complex GINS protein SLD5",
  "term_id": "UNKNOWN:0001"
}